{
  "gene": "UniProtKB:P05014",
  "gene_symbol": "IFNA4",
  "term_label": "cytokine activity",
  "term_id": "GO:0005125",
  "gene_name": "Interferon alpha-4"
}